{
  "gene_name": "Killer cell lectin-like receptor subfamily B member 1",
  "gene": "UniProtKB:Q12918",
  "term_label": "cell surface",
  "term_id": "GO:0009986",
  "gene_symbol": "KLRB1"
}